L-lysine 2,3-aminomutase activity [GO:0050066] (molecular function) Relationships: is_a intramolecular aminotransferase activity [GO:0016869] Sources: RHEA:19177 Also known as: lysine 2,3-aminomutase activity Definition: Catalysis of the reaction: L-lysine = (3S)-3,6-diaminohexanoate.